{
  "gene": "UniProtKB:Q9H019",
  "term_label": "aerobic respiration",
  "gene_symbol": "MTFR1L",
  "term_id": "GO:0009060",
  "gene_name": "Mitochondrial fission regulator 1-like"
}